negative regulation of mitochondrial depolarization [GO:0051902] (biological process) Also known as: down regulation of mitochondrial depolarization, down-regulation of mitochondrial depolarization, downregulation of mitochondrial depolarization, inhibition of mitochondrial depolarization Definition: Any process that stops, prevents, or reduces the frequency, rate or extent of the change in the membrane potential of the mitochondria from negative to positive. Relationships: is a type of regulation of mitochondrial depolarization [GO:0051900]; is a type of negative regulation of membrane depolarization [GO:1904180]; negatively regulates GO:0051882 Sources: GOC:ai